{
  "gene_name": "Cdc42 effector protein 3",
  "gene": "UniProtKB:Q9UKI2",
  "gene_symbol": "CDC42EP3",
  "term_label": "regulation of cell shape",
  "term_id": "GO:0008360"
}